{
  "gene_name": "CCN family member 3",
  "gene": "UniProtKB:P48745",
  "term_label": "extracellular space",
  "term_id": "GO:0005615",
  "gene_symbol": "CCN3"
}